{
  "gene_symbol": "IDE",
  "term_label": "peroxisomal matrix",
  "gene_name": "Insulin-degrading enzyme",
  "term_id": "GO:0005782",
  "gene": "UniProtKB:P14735"
}